TCR signalosome assembly [GO:0036399] (biological process) Also known as: LAT signalosome assembly, linker for activation of T cells signalosome assembly Relationships: is a type of protein-containing complex assembly [GO:0065003] Definition: The aggregation, arrangement and bonding together of a set of components to form a TCR signalosome. References: PMID:22426112 Sources: GOC:krc